{
  "gene_symbol": "SAMD3",
  "gene_name": "Sterile alpha motif domain-containing protein 3",
  "gene": "UniProtKB:Q8N6K7",
  "term_id": "UNKNOWN:0002",
  "term_label": "Unknown biological process"
}